secretory granule maturation [GO:0061792] (biological process) Subtypes: dense core granule maturation [GO:1990502] Relationships: is a type of secretory granule organization [GO:0033363]; is a type of GO:0071695 References: PMID:16618809 Sources: GOC:PARL, GOC:bf, GOC:dph Definition: Steps required to transform an immature secretory vesicle into a mature secretory vesicle. Typically proceeds through homotypic membrane fusion and membrane remodeling.